nuclear proteasome core complex, beta-subunit complex [GO:0031607] (cellular component) Definition: The subunits forming the inner ring of the core complex of a proteasome located in the nucleus of a cell. Relationships: is a type of proteasome core complex, beta-subunit complex [GO:0019774]; is a type of nuclear protein-containing complex [GO:0140513]; is part of nuclear proteasome core complex [GO:0031601] Sources: GOC:mah